{
  "term_id": "GO:0005886",
  "gene_name": "Tetraspanin-12",
  "gene_symbol": "TSPAN12",
  "term_label": "plasma membrane",
  "gene": "UniProtKB:O95859"
}